{
  "term_label": "nucleus",
  "term_id": "GO:0005634",
  "gene_name": "Putative RNA polymerase II subunit B1 CTD phosphatase RPAP2",
  "gene_symbol": "RPAP2",
  "gene": "UniProtKB:Q8IXW5"
}